{
  "gene_symbol": "USP17L15",
  "gene_name": "Ubiquitin carboxyl-terminal hydrolase 17-like protein 15",
  "term_id": "GO:0004843",
  "gene": "UniProtKB:C9J2P7",
  "term_label": "cysteine-type deubiquitinase activity"
}